{
  "gene_name": "Immunoglobulin heavy constant gamma 1",
  "gene_symbol": "IGHG1",
  "term_id": "GO:0019731",
  "term_label": "antibacterial humoral response",
  "gene": "UniProtKB:P01857"
}